negative regulation of hyphopodium formation [GO:0075190] (biological process) Also known as: negative regulation of hyphopodium formation on or near host Relationships: is a type of GO:0051093; is a type of regulation of hyphopodium formation [GO:0075188]; negatively regulates hyphopodium formation [GO:0075187] Sources: GOC:pamgo_curators Definition: Any process that stops, prevents, or reduces the frequency, rate or extent of symbiont hyphopodium formation on or near its host organism. The host is defined as the larger of the organisms involved in a symbiotic interaction.